{
  "gene": "UniProtKB:Q9ULJ6",
  "gene_name": "Zinc finger MIZ domain-containing protein 1",
  "term_id": "GO:0003713",
  "gene_symbol": "ZMIZ1",
  "term_label": "transcription coactivator activity"
}